{
  "term_id": "GO:0005634",
  "gene": "UniProtKB:Q969S2",
  "gene_symbol": "NEIL2",
  "gene_name": "Endonuclease 8-like 2",
  "term_label": "nucleus"
}